{
  "gene_name": "Golgi-specific brefeldin A-resistance guanine nucleotide exchange factor 1",
  "term_id": "GO:0005085",
  "gene": "UniProtKB:Q92538",
  "term_label": "guanyl-nucleotide exchange factor activity",
  "gene_symbol": "GBF1"
}